{
  "gene_name": "Protein FAM87A",
  "gene_symbol": "FAM87A",
  "term_label": "Unknown molecular function",
  "term_id": "UNKNOWN:0001",
  "gene": "UniProtKB:P0C7U9"
}